{
  "gene_name": "Tyrosine-protein kinase Srms",
  "gene_symbol": "SRMS",
  "gene": "UniProtKB:Q9H3Y6",
  "term_label": "non-membrane spanning protein tyrosine kinase activity",
  "term_id": "GO:0004715"
}